{
  "gene": "UniProtKB:Q9UBR2",
  "term_id": "GO:0005764",
  "gene_name": "Cathepsin Z",
  "gene_symbol": "CTSZ",
  "term_label": "lysosome"
}